{
  "gene_symbol": "MFSD10",
  "term_label": "Unknown molecular function",
  "term_id": "UNKNOWN:0001",
  "gene": "UniProtKB:Q14728",
  "gene_name": "Major facilitator superfamily domain-containing protein 10"
}